{
  "gene_symbol": "DMAC2",
  "term_label": "SCF-dependent proteasomal ubiquitin-dependent protein catabolic process",
  "gene_name": "Distal membrane-arm assembly complex protein 2",
  "gene": "UniProtKB:Q9NW81",
  "term_id": "GO:0031146"
}